{
  "term_label": "mitochondrial ribosome",
  "gene": "UniProtKB:Q9BQC6",
  "gene_name": "Large ribosomal subunit protein mL63",
  "term_id": "GO:0005761",
  "gene_symbol": "MRPL57"
}